methyl-ONN-azoxymethanol beta-D-glucosyltransferase activity [GO:0047236] (molecular function) Definition: Catalysis of the reaction: methylazoxymethanol + UDP-D-glucose = H+ + cycasin + UDP. Sources: EC:2.4.1.171, MetaCyc:2.4.1.171-RXN Also known as: methyl-ONN-azoxymethanol glucosyltransferase activity, UDP-glucose:methyl-ONN-azoxymethanol beta-D-glucosyltransferase activity, UDPglucose-methylazoxymethanol glucosyltransferase activity, cycasin synthase activity, uridine diphosphoglucose-methylazoxymethanol glucosyltransferase activity Relationships: is a type of GO:0035251